positive regulation of high-density lipoprotein particle assembly [GO:0090108] (biological process) Definition: Any process that increases the frequency, rate, or extent of high-density lipoprotein particle assembly. High-density lipoprotein particle assembly is the aggregation and arrangement of proteins and lipids to form a high-density lipoprotein particle. Sources: GOC:BHF, GOC:dph, GOC:tb Relationships: is a type of positive regulation of protein-containing complex assembly [GO:0031334]; is a type of GO:0051240; is a type of regulation of high-density lipoprotein particle assembly [GO:0090107]; positively regulates GO:0034380